beta,beta-carotene-9',10'-dioxygenase activity [GO:0050541] (molecular function) Relationships: is_a oxidoreductase activity, acting on the CH-CH group of donors, oxygen as acceptor [GO:0016634] References: PMID:11278918 Also known as: b,b-carotene-9',10'-dioxygenase activity Definition: Catalysis of the reaction: beta-carotene + O2 = beta-apo-10'-carotenal + beta-ionone.